Wnt signaling pathway [GO:0016055] (biological process) Definition: The series of molecular signals initiated by binding of a Wnt protein to a frizzled family receptor on the surface of a target cell and ending with a change in cell state. References: PMID:11532397 Also known as: Wg signaling pathway, Wg signalling pathway, Wingless signaling pathway, Wingless signalling pathway, Wnt receptor signaling pathway, Wnt receptor signalling pathway, frizzled signaling pathway, frizzled signalling pathway, Wnt-activated signaling pathway Relationships: is a type of cell surface receptor signaling pathway [GO:0007166] Subtypes: Wnt signaling pathway involved in heart development [GO:0003306], Wnt signaling pathway involved in forebrain neuroblast division [GO:0021874], non-canonical Wnt signaling pathway [GO:0035567], GO:0060070, Wnt signaling pathway involved in somitogenesis [GO:0090244] Regulation: regulated by GO:0030111; positively regulated by GO:0030177; RO_0002212 by GO:0030178